{
  "gene": "UniProtKB:Q9H223",
  "gene_symbol": "EHD4",
  "term_label": "early endosome",
  "term_id": "GO:0005769",
  "gene_name": "EH domain-containing protein 4"
}